xylan 1,4-beta-xylosidase activity [GO:0009044] (molecular function) Relationships: is a type of xylanase activity [GO:0097599] Sources: EC:3.2.1.37 Definition: Catalysis of the hydrolysis of (1->4)-beta-D-xylans so as to remove successive D-xylose residues from the non-reducing termini. Also known as: 1,4-beta-D-xylan xylohydrolase activity, beta-D-xylopyranosidase activity, beta-xylosidase activity, exo-1,4-beta-D-xylosidase activity, exo-1,4-beta-xylosidase activity, exo-1,4-xylosidase activity, xylobiase activity